CMP phosphorylation [GO:0061566] (biological process) References: PMID:23416111 Sources: GOC:dph Definition: The process of introducing a phosphate group into CMP, cytidine monophosphate, to produce CDP. Addition of two phosphate groups produces CTP. Relationships: is a type of nucleoside monophosphate phosphorylation [GO:0046940]